pyrimidine deoxyribonucleotide catabolic process [GO:0009223] (biological process) Also known as: pyrimidine deoxyribonucleotide breakdown, pyrimidine deoxyribonucleotide catabolism, pyrimidine deoxyribonucleotide degradation Subtypes: dTDP catabolic process [GO:0006246], dCMP catabolic process [GO:0006249], GO:0006251, dCTP catabolic process [GO:0006253], GO:0006257, depyrimidination [GO:0045008], dTMP catabolic process [GO:0046074], GO:0046076, dUMP catabolic process [GO:0046079], dUTP catabolic process [GO:0046081] Sources: GOC:go_curators, ISBN:0198506732 Relationships: is a type of pyrimidine nucleotide catabolic process [GO:0006244]; is a type of GO:0009219; is a type of GO:0009264; is a type of deoxyribose phosphate catabolic process [GO:0046386] Definition: The chemical reactions and pathways resulting in the breakdown of a pyrimidine deoxyribonucleotide, a compound consisting of nucleoside (a pyrimidine base linked to a deoxyribose sugar) esterified with a phosphate group at either the 3' or 5'-hydroxyl group of the sugar.